stress-induced mitochondrial fusion [GO:1990046] (biological process) Definition: Merging of two or more mitochondria within a cell to form a single compartment, as a result of a disturbance in cellular homeostasis. References: PMID:19360003 Sources: GOC:lb Also known as: SIMH, stress-induced mitochondrial hyperfusion, mitochondrial fusion in response to stress Relationships: is a type of mitochondrial fusion [GO:0008053]; is_a cellular response to stress [GO:0033554]